calcium- and calmodulin-responsive adenylate cyclase activity [GO:0008294] (molecular function) Relationships: is a type of adenylate cyclase activity [GO:0004016] References: PMID:1739965 Sources: GOC:mah Also known as: calcium- and calmodulin-responsive adenylyl cyclase activity, calcium/calmodulin-responsive adenylate cyclase activity Definition: Catalysis of the reaction: ATP = 3',5'-cyclic AMP + diphosphate, stimulated by calcium-bound calmodulin.